{
  "gene": "UniProtKB:Q99614",
  "gene_symbol": "TTC1",
  "term_id": "UNKNOWN:0001",
  "gene_name": "Tetratricopeptide repeat protein 1",
  "term_label": "Unknown molecular function"
}